{
  "term_label": "sodium ion transmembrane transport",
  "gene_symbol": "SLC6A3",
  "term_id": "GO:0035725",
  "gene": "UniProtKB:Q01959",
  "gene_name": "Sodium-dependent dopamine transporter"
}